{
  "gene_name": "5-hydroxytryptamine receptor 2B",
  "gene_symbol": "HTR2B",
  "gene": "UniProtKB:P41595",
  "term_id": "GO:0051209",
  "term_label": "release of sequestered calcium ion into cytosol"
}